{
  "term_label": "Unknown molecular function",
  "term_id": "UNKNOWN:0001",
  "gene": "UniProtKB:Q9NSG2",
  "gene_name": "FIGNL1-interacting regulator of recombination and mitosis",
  "gene_symbol": "FIRRM"
}